{
  "gene_name": "Phosphatidylcholine:ceramide cholinephosphotransferase 2",
  "gene_symbol": "SGMS2",
  "term_id": "GO:0005789",
  "term_label": "endoplasmic reticulum membrane",
  "gene": "UniProtKB:Q8NHU3"
}